racemase and epimerase activity [GO:0016854] (molecular function) Subtypes: GO:0004493, GO:0008111, dihydroneopterin triphosphate 2'-epimerase activity [GO:0008719], racemase and epimerase activity, acting on amino acids and derivatives [GO:0016855], racemase and epimerase activity, acting on hydroxy acids and derivatives [GO:0016856], racemase and epimerase activity, acting on carbohydrates and derivatives [GO:0016857], GO:0036348, 16-hydroxysteroid epimerase activity [GO:0047524], allantoin racemase activity [GO:0047653], NAD(P)HX epimerase activity [GO:0052856] Relationships: is a type of GO:0016853 Sources: GOC:mah, ISBN:0198506732 Definition: Catalysis of a reaction that alters the configuration of one or more chiral centers in a molecule. Note: Note that 'epimerase' refers to the conversion of an epimer into its diastereoisomer, and 'racemase' refers to the interconversion of the two enantiomers of a chiral compound. Also known as: racemase and epimerase activity, acting on other compounds